retrograde trans-synaptic signaling by soluble gas [GO:0098923] (biological process) Sources: GOC:dos Relationships: is a type of retrograde trans-synaptic signaling [GO:0098917]; is a type of GO:0099543 Definition: Cell-cell signaling from postsynapse to presynapse, across the synaptic cleft, mediated by an soluble gas ligand. Subtypes: retrograde trans-synaptic signaling by nitric oxide [GO:0098924]